{
  "gene_name": "DNA-binding protein RFX2",
  "term_id": "GO:0005634",
  "gene": "UniProtKB:P48378",
  "term_label": "nucleus",
  "gene_symbol": "RFX2"
}